{
  "term_label": "ubiquitin protein ligase activity",
  "gene_name": "E3 ubiquitin-protein ligase RNF217",
  "term_id": "GO:0061630",
  "gene_symbol": "RNF217",
  "gene": "UniProtKB:Q8TC41"
}